{
  "term_label": "CURI complex",
  "gene": "UniProtKB:Q9H6R4",
  "gene_symbol": "NOL6",
  "term_id": "GO:0032545",
  "gene_name": "Nucleolar protein 6"
}